{
  "gene_name": "Succinate--CoA ligase [ADP_GDP-forming] subunit alpha, mitochondrial",
  "term_label": "tricarboxylic acid cycle",
  "gene_symbol": "SUCLG1",
  "term_id": "GO:0006099",
  "gene": "UniProtKB:P53597"
}